{
  "gene_name": "Dystrotelin",
  "gene": "UniProtKB:A2CJ06",
  "term_label": "synaptic signaling",
  "gene_symbol": "DYTN",
  "term_id": "GO:0099536"
}